sucrose biosynthetic process [GO:0005986] (biological process) Relationships: is a type of GO:0005985; is a type of GO:0046351 Sources: GOC:go_curators Definition: The chemical reactions and pathways resulting in the formation of sucrose, the disaccharide fructofuranosyl-glucopyranoside. Also known as: sucrose anabolism, sucrose biosynthesis, sucrose formation, sucrose synthesis